{
  "gene_name": "Defensin alpha 4",
  "gene_symbol": "DEFA4",
  "term_id": "GO:0050829",
  "gene": "UniProtKB:P12838",
  "term_label": "defense response to Gram-negative bacterium"
}